{
  "term_id": "GO:0007265",
  "term_label": "Ras protein signal transduction",
  "gene_symbol": "DOK2",
  "gene": "UniProtKB:O60496",
  "gene_name": "Docking protein 2"
}